{
  "gene_symbol": "STX7",
  "term_label": "SNARE binding",
  "gene": "UniProtKB:O15400",
  "gene_name": "Syntaxin-7",
  "term_id": "GO:0000149"
}